dopamine biosynthetic process [GO:0042416] (biological process) Regulation: regulated by regulation of dopamine biosynthetic process [GO:1903179]; negatively regulated by negative regulation of dopamine biosynthetic process [GO:1903180]; RO_0002213 by positive regulation of dopamine biosynthetic process [GO:1903181] Relationships: is a type of GO:0042417; is a type of catecholamine biosynthetic process [GO:0042423] Subtypes: dopamine biosynthetic process from tyrosine [GO:0006585] Definition: The chemical reactions and pathways resulting in the formation of dopamine, a catecholamine neurotransmitter and a metabolic precursor of noradrenaline and adrenaline. Sources: GOC:jl, ISBN:0198506732 Also known as: dopamine anabolism, dopamine biosynthesis, dopamine formation, dopamine synthesis